{
  "gene_symbol": "ZNF561",
  "gene_name": "Zinc finger protein 561",
  "term_id": "GO:0000981",
  "term_label": "DNA-binding transcription factor activity, RNA polymerase II-specific",
  "gene": "UniProtKB:Q8N587"
}